{
  "gene_name": "Interstitial collagenase",
  "term_id": "GO:0004222",
  "gene": "UniProtKB:P03956",
  "gene_symbol": "MMP1",
  "term_label": "metalloendopeptidase activity"
}